pyrimidine nucleoside triphosphate metabolic process [GO:0009147] (biological process) Relationships: is_a nucleoside triphosphate metabolic process [GO:0009141] Subtypes: pyrimidine nucleoside triphosphate biosynthetic process [GO:0009148], pyrimidine nucleoside triphosphate catabolic process [GO:0009149], pyrimidine ribonucleoside triphosphate metabolic process [GO:0009208], pyrimidine deoxyribonucleoside triphosphate metabolic process [GO:0009211] Also known as: pyrimidine nucleoside triphosphate metabolism Sources: GOC:go_curators, ISBN:0198506732 Definition: The chemical reactions and pathways involving pyrimidine nucleoside triphosphate, a compound consisting of a pyrimidine base linked to a ribose or deoxyribose sugar esterified with triphosphate on the sugar.